maturation of 2S rRNA [GO:0000475] (biological process) Definition: Any process involved in the maturation of a precursor 2S ribosomal RNA (rRNA) molecule into a mature 2S rRNA molecule. Sources: GOC:curators Relationships: is a type of rRNA processing [GO:0006364]